ferric-hydroxamate import into cell [GO:0015687] (biological process) Also known as: ferric-hydroxamate transport Relationships: is a type of siderophore-iron import into cell [GO:0033214] Definition: A process in which ferric-hydroxamate, the iron-bound form of the iron chelator hydroxamate, is transported into the cell by specific cell surface receptors. Subtypes: GO:0042928 References: PMID:23192658 Sources: GOC:pg